NHE3/E3KARP/ACTN4 complex [GO:0032766] (cellular component) Relationships: is a type of protein-containing complex [GO:0032991] References: PMID:11948184 Also known as: NHE3/E3KARP/alpha-actinin complex Definition: A heterotrimeric protein complex formed by the association of NHE3, E3KARP and alpha-actinin upon an increase in calcium ion concentration; found in clusters localized on plasma membrane and in intracellular compartments.